regulation of Wnt-Frizzled-LRP5/6 complex assembly [GO:1904711] (biological process) Also known as: regulation of Wnt receptor complex assembly, regulation of Wnt-FZD-LRP5/6 trimeric complex assembly, regulation of Wnt-FZD-LRP5/6 trimeric complex formation, regulation of WNT-FZD-LRP5 complex assembly, regulation of WNT-FZD-LRP5 complex formation, regulation of WNT-FZD-LRP6 complex assembly, regulation of WNT-FZD-LRP6 complex formation, regulation of Frizzled-LRP5/6 complex assembly, regulation of Frizzled-LRP5/6 complex formation, regulation of Wnt-induced Frizzled-LRP5/6 complex assembly, regulation of Wnt-induced Frizzled-LRP5/6 complex formation Relationships: is a type of regulation of protein-containing complex assembly [GO:0043254]; regulates GO:1904701 Subtypes: positive regulation of Wnt-Frizzled-LRP5/6 complex assembly [GO:1904712], GO:1904723 Definition: Any process that modulates the frequency, rate or extent of Wnt-Frizzled-LRP5/6 complex assembly. Sources: GOC:PARL, GOC:TermGenie, GOC:bf, GO_REF:0000058